{
  "gene_symbol": "DNM2",
  "gene_name": "Dynamin-2",
  "gene": "UniProtKB:P50570",
  "term_id": "GO:0003924",
  "term_label": "GTPase activity"
}